{
  "gene_symbol": "TAF5L",
  "term_label": "regulation of DNA-templated transcription",
  "term_id": "GO:0006355",
  "gene": "UniProtKB:O75529",
  "gene_name": "TAF5-like RNA polymerase II p300_CBP-associated factor-associated factor 65 kDa subunit 5L"
}